{
  "term_label": "positive regulation of tumor necrosis factor production",
  "gene_name": "Toll_interleukin-1 receptor domain-containing adapter protein",
  "gene_symbol": "TIRAP",
  "gene": "UniProtKB:P58753",
  "term_id": "GO:0032760"
}